{
  "term_id": "GO:0006338",
  "gene_symbol": "ACTL6B",
  "term_label": "chromatin remodeling",
  "gene_name": "Actin-like protein 6B",
  "gene": "UniProtKB:O94805"
}